{
  "gene_name": "Amphiregulin",
  "term_label": "positive regulation of cell population proliferation",
  "gene": "UniProtKB:P15514",
  "gene_symbol": "AREG",
  "term_id": "GO:0008284"
}